double strand break-nuclear membrane anchor activity [GO:0062241] (molecular function) Definition: Binding to DNA double strand breaks and the nuclear inner membrane, in order to facilitate DNA repair. Relationships: is a type of protein-membrane adaptor activity [GO:0043495] Also known as: DNA repair factory References: PMID:31635174